cytidylate cyclase activity [GO:0047805] (molecular function) Also known as: 3',5'-cyclic-CMP synthase activity, 3'5'-cyclic-CMP synthase activity, CTP diphosphate-lyase (cyclizing), CTP diphosphate-lyase (cyclizing; 3',5'-cyclic-CMP-forming), cytidyl cyclase activity, cytidylyl cyclase activity Sources: RHEA:14737 Relationships: is a type of cyclase activity [GO:0009975]; is a type of GO:0016849; is part of GO:0009190 Definition: Catalysis of the reaction: CTP = 3',5'-cyclic CMP + diphosphate + H+.